{
  "gene_symbol": "ZBED3",
  "term_id": "UNKNOWN:0003",
  "gene": "UniProtKB:Q96IU2",
  "term_label": "Unknown cellular component",
  "gene_name": "Zinc finger BED domain-containing protein 3"
}